{
  "gene_symbol": "C9orf72",
  "term_label": "autophagy",
  "gene": "UniProtKB:Q96LT7",
  "gene_name": "Guanine nucleotide exchange factor C9orf72",
  "term_id": "GO:0006914"
}